very-long-chain enoyl-CoA reductase activity [GO:0102758] (molecular function) Definition: Catalysis of the reaction: a very-long-chain 2,3-saturated fatty acyl-CoA + NADP+ = a very-long-chain (2E)-enoyl-CoA + H+ + NADPH. This reaction is the fourth (reduction) step of the four-step fatty acid elongation cycle in the endoplasmic reticulum that extends fatty acids of C-16 or longer with an additional 2-C unit. References: PMID:16564093, PMID:19763486 Sources: RHEA:14473 Relationships: is a type of oxidoreductase activity, acting on the CH-CH group of donors, NAD or NADP as acceptor [GO:0016628]